{
  "term_label": "Unknown cellular component",
  "gene_symbol": "CNPY4",
  "term_id": "UNKNOWN:0003",
  "gene": "UniProtKB:Q8N129",
  "gene_name": "Protein canopy homolog 4"
}